regulation of ductus arteriosus closure [GO:1904335] (biological process) References: PMID:16303610 Sources: GOC:TermGenie, GO_REF:0000058 Definition: Any process that modulates the frequency, rate or extent of ductus arteriosus closure. Relationships: is a type of regulation of artery morphogenesis [GO:1905651]; regulates ductus arteriosus closure [GO:0097070] Subtypes: negative regulation of ductus arteriosus closure [GO:1904336], GO:1904337